{
  "gene_name": "Zinc finger protein 337",
  "gene": "UniProtKB:Q9Y3M9",
  "gene_symbol": "ZNF337",
  "term_id": "GO:0005634",
  "term_label": "nucleus"
}